{
  "term_label": "antifungal innate immune response",
  "term_id": "GO:0061760",
  "gene_symbol": "CLEC4A",
  "gene": "UniProtKB:Q9UMR7",
  "gene_name": "C-type lectin domain family 4 member A"
}